{
  "gene_symbol": "RIGI",
  "term_id": "GO:0002753",
  "gene": "UniProtKB:O95786",
  "term_label": "cytoplasmic pattern recognition receptor signaling pathway",
  "gene_name": "Antiviral innate immune response receptor RIG-I"
}